{
  "term_id": "GO:0019509",
  "gene_name": "Methylthioribulose-1-phosphate dehydratase",
  "gene": "UniProtKB:Q96GX9",
  "term_label": "L-methionine salvage from methylthioadenosine",
  "gene_symbol": "APIP"
}